{
  "gene": "UniProtKB:A6NNZ2",
  "gene_name": "Tubulin beta 8B",
  "gene_symbol": "TUBB8B",
  "term_label": "cytoplasm",
  "term_id": "GO:0005737"
}